{
  "gene": "UniProtKB:O75419",
  "gene_symbol": "CDC45",
  "term_id": "GO:0003697",
  "term_label": "single-stranded DNA binding",
  "gene_name": "Cell division control protein 45 homolog"
}